{
  "gene_symbol": "UCK1",
  "term_label": "cytoplasm",
  "gene": "UniProtKB:Q9HA47",
  "gene_name": "Uridine-cytidine kinase 1",
  "term_id": "GO:0005737"
}